{
  "term_id": "GO:0005886",
  "term_label": "plasma membrane",
  "gene": "UniProtKB:O14526",
  "gene_symbol": "FCHO1",
  "gene_name": "F-BAR domain only protein 1"
}